{
  "gene_symbol": "SPATA7",
  "term_id": "GO:0000226",
  "gene": "UniProtKB:Q9P0W8",
  "gene_name": "Spermatogenesis-associated protein 7",
  "term_label": "microtubule cytoskeleton organization"
}